{
  "gene": "UniProtKB:Q5TA82",
  "gene_symbol": "LCE2D",
  "gene_name": "Late cornified envelope protein 2D",
  "term_label": "Unknown cellular component",
  "term_id": "UNKNOWN:0003"
}